{
  "gene": "UniProtKB:O15247",
  "gene_symbol": "CLIC2",
  "term_id": "GO:0005737",
  "gene_name": "Chloride intracellular channel protein 2",
  "term_label": "cytoplasm"
}